renal zinc excretion [GO:0180002] (biological process) Relationships: is a type of renal tubular secretion [GO:0097254] Also known as: renal zinc ion excretion, renal zinc secretion Definition: The elimination of zinc ions from peritubular capillaries (or surrounding hemolymph in invertebrates) into the renal tubules to be incorporated subsequently into the urine. References: PMID:28196538